{
  "term_id": "UNKNOWN:0001",
  "gene": "UniProtKB:Q86TZ1",
  "gene_name": "Tetratricopeptide repeat protein 6",
  "gene_symbol": "TTC6",
  "term_label": "Unknown molecular function"
}